{
  "gene_symbol": "CBS",
  "gene": "UniProtKB:P35520",
  "gene_name": "Cystathionine beta-synthase",
  "term_id": "GO:0006535",
  "term_label": "cysteine biosynthetic process from serine"
}